heme import across plasma membrane [GO:1904334] (biological process) Also known as: heme assimilation Definition: The directed movement of heme from outside of a cell, across the plasma membrane and into the cytosol. References: PMID:25733668 Sources: GOC:TermGenie, GO_REF:0000075 Relationships: is a type of heme transmembrane transport [GO:0035351]; is a type of iron ion import across plasma membrane [GO:0098711]; is a type of heme import into cell [GO:0140420]